{
  "term_label": "positive regulation of transcription by RNA polymerase II",
  "gene_symbol": "ABHD14B",
  "term_id": "GO:0045944",
  "gene": "UniProtKB:Q96IU4",
  "gene_name": "Putative protein-lysine deacylase ABHD14B"
}